UDP-galactopyranose mutase activity [GO:0008767] (molecular function) Also known as: UDP-D-galactopyranose furanomutase activity, UDPgalactopyranose mutase activity Definition: Catalysis of the reaction: UDP-D-galactopyranose = UDP-D-galacto-1,4-furanose. Sources: EC:5.4.99.9 Relationships: is a type of GO:0016866